{
  "gene": "UniProtKB:A8MUM7",
  "term_label": "Unknown cellular component",
  "gene_name": "Galectin-16",
  "term_id": "UNKNOWN:0003",
  "gene_symbol": "LGALS16"
}